negative stranded viral RNA replication [GO:0039689] (biological process) Definition: A viral genome replication process where the template genome is negative stranded, single stranded RNA ((-)ssRNA). Also known as: (-)ss viral RNA replication Relationships: is a type of GO:0039694; has part GO:0039696 Sources: GOC:bf, GOC:jl, VZ:1096